{
  "term_id": "GO:0046649",
  "gene_name": "Lymphocyte transmembrane adapter 1",
  "gene": "UniProtKB:Q8IWV1",
  "gene_symbol": "LAX1",
  "term_label": "lymphocyte activation"
}